{
  "term_label": "Unknown cellular component",
  "gene_name": "TM2 domain-containing protein 3",
  "term_id": "UNKNOWN:0003",
  "gene": "UniProtKB:Q9BRN9",
  "gene_symbol": "TM2D3"
}